stele development [GO:0010479] (biological process) Sources: GOC:tb Definition: The process whose specific outcome is the progression of the stele over time, from its formation to the mature structure. The stele is the central column of primary vascular tissue in the root and any tissue that it surrounds. Relationships: is a type of tissue development [GO:0009888]; BFO_0000050 root development [GO:0048364]